photosystem II repair [GO:0010206] (biological process) Sources: GOC:sm Definition: Proteolysis of the damaged D1 protein and re-assembly of a new D1 subunit in the photosystem II following photoinhibition. Relationships: is a type of protein repair [GO:0030091]; is part of photosynthesis, light harvesting [GO:0009765]